{
  "term_id": "UNKNOWN:0003",
  "gene": "UniProtKB:P0CZ25",
  "gene_symbol": "DNAH10OS",
  "gene_name": "Uncharacterized protein DNAH10OS",
  "term_label": "Unknown cellular component"
}